{
  "term_label": "regulation of cytokine production",
  "gene_name": "Zinc finger and BTB domain-containing protein 6",
  "gene_symbol": "ZBTB6",
  "term_id": "GO:0001817",
  "gene": "UniProtKB:Q15916"
}